{
  "gene_symbol": "H2AC8",
  "term_id": "GO:0030527",
  "term_label": "structural constituent of chromatin",
  "gene": "UniProtKB:P04908",
  "gene_name": "Histone H2A type 1-B_E"
}